{
  "gene_symbol": "ZNF256",
  "term_id": "GO:0005634",
  "term_label": "nucleus",
  "gene": "UniProtKB:Q9Y2P7",
  "gene_name": "Zinc finger protein 256"
}